{
  "gene": "UniProtKB:Q13415",
  "gene_name": "Origin recognition complex subunit 1",
  "term_id": "GO:0005664",
  "term_label": "nuclear origin of replication recognition complex",
  "gene_symbol": "ORC1"
}